{
  "gene_name": "Putative protein FAM90A26",
  "gene": "UniProtKB:D6RGX4",
  "gene_symbol": "FAM90A26",
  "term_id": "UNKNOWN:0002",
  "term_label": "Unknown biological process"
}